peptidyl-oxazoline dehydrogenase activity [GO:0018129] (molecular function) Relationships: is a type of oxidoreductase activity, acting on the CH-CH group of donors [GO:0016627] References: PMID:19058272 Sources: GOC:mah Definition: Catalysis of the reduction of a peptide-linked oxazoline to oxazole.